cellular response to tert-butyl hydroperoxide [GO:0072736] (biological process) Definition: Any process that results in a change in state or activity of a cell (in terms of movement, secretion, enzyme production, gene expression, etc.) as a result of a tert-butyl hydroperoxide (t-BOOH) stimulus. Sources: GOC:mah Also known as: cellular response to 2-methyl-prop-2-yl-hydroperoxide, cellular response to t-BOOH Relationships: is a type of cellular response to alkyl hydroperoxide [GO:0071448]; is a type of GO:0072735